{
  "gene_name": "NADH-ubiquinone oxidoreductase chain 6",
  "term_label": "mitochondrion",
  "gene_symbol": "MT-ND6",
  "gene": "UniProtKB:P03923",
  "term_id": "GO:0005739"
}